central nervous system maturation [GO:0021626] (biological process) Relationships: is a type of anatomical structure maturation [GO:0071695]; is part of central nervous system development [GO:0007417] Definition: A developmental process, independent of morphogenetic (shape) change, that is required for the central nervous system to attain its fully functional state. The central nervous system is the core nervous system that serves an integrating and coordinating function. In vertebrates it consists of the brain and spinal cord. In those invertebrates with a central nervous system it typically consists of a brain, cerebral ganglia and a nerve cord. Sources: GOC:cls, GOC:dgh, GOC:dph, GOC:jid, GO_REF:0000021